{
  "gene_name": "Histone acetyltransferase p300",
  "gene_symbol": "EP300",
  "term_id": "GO:0031490",
  "term_label": "chromatin DNA binding",
  "gene": "UniProtKB:Q09472"
}